{
  "term_id": "GO:0045202",
  "gene_name": "Receptor-type tyrosine-protein phosphatase-like N",
  "term_label": "synapse",
  "gene_symbol": "PTPRN",
  "gene": "UniProtKB:Q16849"
}